{
  "term_id": "GO:0005634",
  "term_label": "nucleus",
  "gene_name": "PAX3- and PAX7-binding protein 1",
  "gene_symbol": "PAXBP1",
  "gene": "UniProtKB:Q9Y5B6"
}